{
  "gene_symbol": "IGLV3-21",
  "term_id": "UNKNOWN:0001",
  "gene_name": "Immunoglobulin lambda variable 3-21",
  "term_label": "Unknown molecular function",
  "gene": "UniProtKB:P80748"
}